{
  "gene_symbol": "XG",
  "gene": "UniProtKB:P55808",
  "term_label": "Unknown molecular function",
  "gene_name": "Glycoprotein Xg",
  "term_id": "UNKNOWN:0001"
}